{
  "gene_symbol": "ZNF24",
  "term_id": "UNKNOWN:0003",
  "term_label": "Unknown cellular component",
  "gene_name": "Zinc finger protein 24",
  "gene": "UniProtKB:P17028"
}